{
  "gene_symbol": "ARMC1",
  "gene_name": "Armadillo repeat-containing protein 1",
  "gene": "UniProtKB:Q9NVT9",
  "term_id": "UNKNOWN:0002",
  "term_label": "Unknown biological process"
}